{
  "gene_symbol": "SORBS2",
  "term_id": "GO:0007010",
  "gene": "UniProtKB:O94875",
  "gene_name": "Sorbin and SH3 domain-containing protein 2",
  "term_label": "cytoskeleton organization"
}